{
  "term_label": "cytoplasm",
  "gene_name": "Lethal(2) giant larvae protein homolog 1",
  "gene_symbol": "LLGL1",
  "term_id": "GO:0005737",
  "gene": "UniProtKB:Q15334"
}